trimethylamine-oxide aldolase activity [GO:0050352] (MF) Sources: EC:4.1.2.32, RHEA:20217 Also known as: trimethylamine N-oxide aldolase activity, trimethylamine N-oxide demethylase activity, trimethylamine N-oxide formaldehyde-lyase activity, trimethylamine-N-oxide formaldehyde-lyase (dimethylamine-forming), trimethylamine-N-oxide formaldehyde-lyase activity Definition: Catalysis of the reaction: H+ + trimethylamine N-oxide = dimethylamine + formaldehyde. Relationships: is a type of aldehyde-lyase activity [GO:0016832]